{
  "gene": "UniProtKB:Q9GZY6",
  "term_label": "B cell activation",
  "term_id": "GO:0042113",
  "gene_symbol": "LAT2",
  "gene_name": "Linker for activation of T-cells family member 2"
}